{
  "gene": "UniProtKB:P23468",
  "term_id": "GO:0007165",
  "gene_symbol": "PTPRD",
  "gene_name": "Receptor-type tyrosine-protein phosphatase delta",
  "term_label": "signal transduction"
}